{
  "gene_symbol": "USP39",
  "term_id": "GO:0000245",
  "term_label": "spliceosomal complex assembly",
  "gene": "UniProtKB:Q53GS9",
  "gene_name": "U4_U6.U5 tri-snRNP-associated protein 2"
}